positive regulation of apoptotic signaling pathway [GO:2001235] (biological process) Relationships: is a type of positive regulation of signal transduction [GO:0009967]; is a type of GO:0043065; is a type of GO:2001233; positively regulates apoptotic signaling pathway [GO:0097190] Also known as: positive regulation of apoptotic signalling pathway Sources: GOC:mtg_apoptosis Subtypes: GO:2001238, GO:2001244 Definition: Any process that activates or increases the frequency, rate or extent of apoptotic signaling pathway.